L-glutamate catabolic process to butyrate [GO:0033508] (biological process) Subtypes: L-glutamate catabolic process via 2-hydroxyglutarate [GO:0019552] Also known as: glutamate breakdown to butyrate, glutamate degradation to butyrate Relationships: is a type of L-glutamate catabolic process [GO:0006538]; is a type of butyrate metabolic process [GO:0019605] Definition: The chemical reactions and pathways resulting in the breakdown of L-glutamate into other compounds, including butyrate. Sources: GOC:mah, MetaCyc:PWY-5087